EmrE multidrug transporter complex [GO:1990207] (cellular component) Also known as: EmrE complex References: PMID:18024586 Sources: GOC:bhm Definition: A transmembrane protein complex capable of transporting positively charged hydrophobic drugs across the plasma membrane thereby involved in conferring resistance to a wide range of toxic compounds (e.g. methyl viologen, ethidium bromide and acriflavine). It is commonly found in bacteria. In E. coli it forms a homodimer. Relationships: is a type of plasma membrane protein complex [GO:0098797]; is a type of transmembrane transporter complex [GO:1902495]